response to parasitic plant [GO:0002241] (biological process) Definition: Any process that results in a change in state or activity of a cell or an organism (in terms of movement, secretion, enzyme production, gene expression, etc.) as a result of a stimulus from a parasitic plant. Subtypes: GO:0002242, detection of parasitic plant [GO:0002243] References: PMID:16547862 Sources: GOC:add Relationships: is a type of response to symbiont [GO:0009608]